{
  "gene": "UniProtKB:Q5VW38",
  "gene_name": "Protein GPR107",
  "term_label": "clathrin-coated vesicle",
  "term_id": "GO:0030136",
  "gene_symbol": "GPR107"
}